spermidine transmembrane transporter activity [GO:0015606] (molecular function) Definition: Enables the transfer of spermidine, N-(3-aminopropyl)-1,4-diaminobutane, from one side of a membrane to the other. Sources: GOC:ai Relationships: is_a polyamine transmembrane transporter activity [GO:0015203]; is part of spermidine transmembrane transport [GO:1903711]